{
  "gene": "UniProtKB:Q6H3X3",
  "term_id": "GO:0002486",
  "gene_name": "UL-16 binding protein 5",
  "term_label": "antigen processing and presentation of endogenous peptide antigen via MHC class I via ER pathway, TAP-independent",
  "gene_symbol": "RAET1G"
}